{
  "gene_name": "Steryl-sulfatase",
  "gene_symbol": "STS",
  "term_label": "Unknown cellular component",
  "term_id": "UNKNOWN:0003",
  "gene": "UniProtKB:P08842"
}